4-hydroxyphenylpyruvate decarboxylase activity [GO:0050546] (molecular function) Sources: EC:4.1.1.80, RHEA:18697 Also known as: 4-hydroxyphenylpyruvate carboxy-lyase (4-hydroxyphenylacetaldehyde-forming), 4-hydroxyphenylpyruvate carboxy-lyase activity Definition: Catalysis of the reaction: (4-hydroxyphenyl)pyruvate + H+ = (4-hydroxyphenyl)acetaldehyde + CO2. Relationships: is a type of carboxy-lyase activity [GO:0016831]